{
  "gene": "UniProtKB:Q6ZTW0",
  "gene_name": "Tubulin polyglutamylase complex subunit 1",
  "term_label": "tubulin-glutamic acid ligase activity",
  "term_id": "GO:0070740",
  "gene_symbol": "TPGS1"
}